{
  "term_label": "DNA-templated DNA replication",
  "gene": "UniProtKB:P28340",
  "term_id": "GO:0006261",
  "gene_name": "DNA polymerase delta catalytic subunit",
  "gene_symbol": "POLD1"
}